{
  "term_id": "GO:0005794",
  "gene_symbol": "IFT27",
  "term_label": "Golgi apparatus",
  "gene_name": "Intraflagellar transport protein 27 homolog",
  "gene": "UniProtKB:Q9BW83"
}